{
  "gene": "UniProtKB:Q16514",
  "gene_name": "Transcription initiation factor TFIID subunit 12",
  "term_label": "TBP-class protein binding",
  "term_id": "GO:0017025",
  "gene_symbol": "TAF12"
}